{
  "gene": "UniProtKB:Q9BQE6",
  "term_id": "GO:0005634",
  "gene_symbol": "LBHD1",
  "gene_name": "LBH domain-containing protein 1",
  "term_label": "nucleus"
}